{
  "gene_name": "Disintegrin and metalloproteinase domain-containing protein 33",
  "gene_symbol": "ADAM33",
  "term_label": "proteolysis",
  "term_id": "GO:0006508",
  "gene": "UniProtKB:Q9BZ11"
}